host-mediated perturbation of viral transcription [GO:0043921] (BP) Relationships: is a type of host-mediated perturbation of viral process [GO:0044788] Also known as: modulation by host of viral transcription, regulation by host of viral transcription, regulation of viral transcription by host Definition: A process in which a host organism alters or subverts viral transcription. Sources: GOC:jl Subtypes: host-mediated suppression of viral transcription [GO:0043922], GO:0043923